{
  "gene": "UniProtKB:Q02575",
  "gene_name": "Helix-loop-helix protein 1",
  "term_label": "regulation of transcription by RNA polymerase II",
  "gene_symbol": "NHLH1",
  "term_id": "GO:0006357"
}